{
  "term_label": "Unknown biological process",
  "gene_symbol": "THNSL1",
  "gene": "UniProtKB:Q8IYQ7",
  "gene_name": "Threonine synthase-like 1",
  "term_id": "UNKNOWN:0002"
}